{
  "term_label": "Unknown cellular component",
  "term_id": "UNKNOWN:0003",
  "gene": "UniProtKB:Q15283",
  "gene_name": "Ras GTPase-activating protein 2",
  "gene_symbol": "RASA2"
}